{
  "term_id": "GO:0003729",
  "gene_name": "RNA-binding protein 4B",
  "gene_symbol": "RBM4B",
  "gene": "UniProtKB:Q9BQ04",
  "term_label": "mRNA binding"
}